{
  "gene_name": "Translation initiation factor eIF-2B subunit delta",
  "term_id": "GO:0002183",
  "term_label": "cytoplasmic translational initiation",
  "gene": "UniProtKB:Q9UI10",
  "gene_symbol": "EIF2B4"
}